{
  "term_label": "keratin filament",
  "term_id": "GO:0045095",
  "gene_name": "Keratin, type I cytoskeletal 13",
  "gene": "UniProtKB:P13646",
  "gene_symbol": "KRT13"
}